ecdysteroid 22-hydroxylase activity [GO:0042767] (molecular function) Also known as: 3-dehydro-2,22-dideoxyecdysone 22-hydroxylase activity Relationships: is a type of steroid hydroxylase activity [GO:0008395]; is a type of oxidoreductase activity, acting on paired donors, with incorporation or reduction of molecular oxygen, reduced iron-sulfur protein as one donor, and incorporation of one atom of oxygen [GO:0016713] Definition: Catalysis of the reaction: 3-dehydro-2,22-dideoxyecdysone + 2 reduced [adrenodoxin] + O2 + 2 H+ = 3-dehydro-2-deoxyecdysone + 2 oxidized [adrenodoxin] + H2O. Other substrates include 3-dehydro-2,22,25-deoxyecdysone and 2,22-dideoxyecdysone. References: PMID:12177427 Sources: EC:1.14.15.44